{
  "gene_symbol": "ABCA9",
  "gene": "UniProtKB:Q8IUA7",
  "term_label": "ATPase-coupled transmembrane transporter activity",
  "term_id": "GO:0042626",
  "gene_name": "ATP-binding cassette sub-family A member 9"
}